cellular response to corticosterone stimulus [GO:0071386] (BP) Relationships: is a type of response to corticosterone [GO:0051412]; is_a cellular response to glucocorticoid stimulus [GO:0071385]; is a type of cellular response to mineralocorticoid stimulus [GO:0071389]; is_a GO:0097306; is a type of cellular response to ketone [GO:1901655] Sources: GOC:mah Definition: Any process that results in a change in state or activity of a cell (in terms of movement, secretion, enzyme production, gene expression, etc.) as a result of a corticosterone stimulus. Corticosterone is a 21 carbon steroid hormone of the corticosteroid type, produced in the cortex of the adrenal glands. In many species, corticosterone is the principal glucocorticoid, involved in regulation of fuel metabolism, immune reactions, and stress responses.